peripheral tolerance induction to self antigen [GO:0002466] (biological process) Sources: GOC:jal, ISBN:0781735149 Relationships: is a type of peripheral tolerance induction [GO:0002465]; is a type of tolerance induction to self antigen [GO:0002513] Definition: Tolerance induction to self antigens in the peripheral lymphoid tissues: blood, lymph nodes, spleen, and mucosal-associated lymphoid tissues.